{
  "gene_symbol": "FAM72D",
  "gene": "UniProtKB:Q6L9T8",
  "term_id": "UNKNOWN:0001",
  "term_label": "Unknown molecular function",
  "gene_name": "Protein FAM72D"
}